{
  "gene_symbol": "VSNL1",
  "gene_name": "Visinin-like protein 1",
  "term_id": "UNKNOWN:0003",
  "term_label": "Unknown cellular component",
  "gene": "UniProtKB:P62760"
}